anthocyanidin reductase activity [GO:0033729] (molecular function) Definition: Catalysis of the reaction: a flavan-3-ol + 2 NAD(P)+ = an anthocyanidin + 2 NAD(P)H + H+. Relationships: is a type of oxidoreductase activity, acting on the CH-CH group of donors, NAD or NADP as acceptor [GO:0016628] Also known as: ANR, AtANR, MtANR, flavan-3-ol:NAD(P)+ oxidoreductase activity Sources: EC:1.3.1.77